{
  "term_id": "GO:0005634",
  "gene": "UniProtKB:P11473",
  "gene_name": "Vitamin D3 receptor",
  "gene_symbol": "VDR",
  "term_label": "nucleus"
}